positive regulation of cardiac muscle tissue regeneration [GO:1905180] (biological process) Also known as: up regulation of cardiac muscle tissue regeneration, up-regulation of cardiac muscle tissue regeneration, upregulation of cardiac muscle tissue regeneration, activation of cardiac muscle tissue regeneration Relationships: is a type of GO:0048639; is a type of regulation of cardiac muscle tissue regeneration [GO:1905178]; positively regulates cardiac muscle tissue regeneration [GO:0061026] References: PMID:23222520 Sources: GOC:BHF, GOC:BHF_miRNA, GOC:TermGenie, GOC:rph, GO_REF:0000058 Definition: Any process that activates or increases the frequency, rate or extent of cardiac muscle tissue regeneration.